{
  "term_label": "transforming growth factor beta binding",
  "gene_name": "WAP, Kazal, immunoglobulin, Kunitz and NTR domain-containing protein 1",
  "gene": "UniProtKB:Q96NZ8",
  "gene_symbol": "WFIKKN1",
  "term_id": "GO:0050431"
}